dinoflagellate sulcal notch [GO:0097618] (cellular component) Definition: A dinoflagellate sulcus that extends all the way to the posterior end of the cell (also known as antapex). The presence of a sulcal notch makes the dinoflagellate hypocone appear bilobed. References: PMID:7002229 Sources: GOC:at, Wikipedia:Dinoflagellate#Morphology, http://tolweb.org/Dinoflagellates/2445 Note: The term name refers to a taxonomic group to make the label unique with respect to similarly-named anatomical structures. Also, the ventral (front) side of a dinoflagellate cell is the one where the sulcus is located (as opposed to the dorsal (back) side). The term 'sulcal notch' appears mostly in older literature; more recently, indication of a bilobed hypocone is used to express the same. Also known as: dinoflagellate sulcus notch, sulcal notch Relationships: is a type of dinoflagellate sulcus [GO:0097612]